{
  "term_label": "nucleus",
  "gene_symbol": "TCIM",
  "term_id": "GO:0005634",
  "gene": "UniProtKB:Q9NR00",
  "gene_name": "Transcriptional and immune response regulator"
}